{
  "term_label": "proteasome-mediated ubiquitin-dependent protein catabolic process",
  "gene_name": "Kelch-like protein 41",
  "gene_symbol": "KLHL41",
  "term_id": "GO:0043161",
  "gene": "UniProtKB:O60662"
}